{
  "term_label": "phosphatidylinositol 3-kinase/protein kinase B signal transduction",
  "gene_symbol": "PIK3CB",
  "gene": "UniProtKB:P42338",
  "gene_name": "Phosphatidylinositol 4,5-bisphosphate 3-kinase catalytic subunit beta isoform",
  "term_id": "GO:0043491"
}